{
  "gene": "UniProtKB:Q9UNQ0",
  "gene_name": "Broad substrate specificity ATP-binding cassette transporter ABCG2",
  "gene_symbol": "ABCG2",
  "term_label": "transmembrane transport",
  "term_id": "GO:0055085"
}